establishment of floral organ orientation [GO:0048559] (biological process) Relationships: is a type of GO:0003006; is a type of GO:0090707; is part of GO:0048439 Sources: GOC:jid Definition: The process that determines the orientation of the floral organs with reference to the central axis of the flower. Subtypes: GO:0048498